{
  "term_id": "GO:0048705",
  "gene": "UniProtKB:Q2UY09",
  "term_label": "skeletal system morphogenesis",
  "gene_symbol": "COL28A1",
  "gene_name": "Collagen alpha-1(XXVIII) chain"
}